specification of segmental identity, mandibular segment [GO:0042305] (biological process) Relationships: is a type of specification of segmental identity, head [GO:0007380]; is part of GO:0035289 Sources: ISBN:0878932437 Definition: The specification of the characteristic structures of the mandibular segment following establishment of segment boundaries. Identity is considered to be the aggregate of characteristics by which a structure is recognized. Note: See also the fly_anatomy.ontology term 'mandibular segment ; FBbt:00000012'.